{
  "gene_name": "Matrix metalloproteinase-27",
  "term_label": "Unknown cellular component",
  "gene": "UniProtKB:Q9H306",
  "term_id": "UNKNOWN:0003",
  "gene_symbol": "MMP27"
}